{
  "gene_name": "Alpha-tocopherol transfer protein-like",
  "gene_symbol": "TTPAL",
  "gene": "UniProtKB:Q9BTX7",
  "term_label": "Unknown cellular component",
  "term_id": "UNKNOWN:0003"
}